dol-P-Man:Man(7)GlcNAc(2)-PP-Dol alpha-1,6-mannosyltransferase activity [GO:0052917] (MF) Also known as: dolichyl-P-mannose:Man(7)GlcNAc(2)-PP-dolichyl mannosyltransferase activity, dolichyl-pyrophosphate Man7GlcNAc2 alpha-1,6-mannosyltransferase activity Relationships: is a type of alpha-1,6-mannosyltransferase activity [GO:0000009]; is a type of GlcNAc(2)-PP-Dol mannosyltransferase activity [GO:0120562] Definition: Catalysis of the reaction: an alpha-D-Man-(1->2)-alpha-D-Man-(1->2)-alpha-D-Man-(1->3)-[alpha-D-Man-(1->2)-alpha-D-Man-(1->3)-alpha-D-Man-(1->6)]-beta-D-Man-(1->4)-beta-D-GlcNAc-(1->4)-alpha-D-GlcNAc-diphospho-di-trans,poly-cis-dolichol + a di-trans,poly-cis-dolichyl beta-D-mannosyl phosphate = an alpha-D-Man-(1->2)-alpha-D-Man-(1->2)-alpha-D-Man-(1->3)-[alpha-D-Man-(1->2)-alpha-D-Man-(1->3)-[alpha-D-Man-(1->6)]-alpha-D-Man-(1->6)]-beta-D-Man-(1->4)-beta-D-GlcNAc-(1->4)-alpha-D-GlcNAc-diphospho-di-trans,poly-cis-dolichol + a di-trans,poly-cis-dolichyl phosphate + H+. References: PMID:10336995 Sources: RHEA:29535